positive regulation of plasma membrane raft polarization [GO:1903908] (biological process) Relationships: is a type of positive regulation of cellular component organization [GO:0051130]; is a type of regulation of plasma membrane raft polarization [GO:1903906]; positively regulates plasma membrane raft polarization [GO:0044858] References: PMID:23575248 Sources: GOC:TermGenie, GOC:als, GO_REF:0000058 Also known as: up regulation of plasma membrane raft polarization, up-regulation of plasma membrane raft polarization, upregulation of plasma membrane raft polarization, activation of plasma membrane raft polarization Definition: Any process that activates or increases the frequency, rate or extent of plasma membrane raft polarization.